{
  "gene_symbol": "MLANA",
  "gene_name": "Melanoma antigen recognized by T-cells 1",
  "term_label": "endoplasmic reticulum membrane",
  "gene": "UniProtKB:Q16655",
  "term_id": "GO:0005789"
}